{
  "term_label": "cytoplasm",
  "gene": "UniProtKB:P63162",
  "gene_symbol": "SNRPN",
  "gene_name": "Small nuclear ribonucleoprotein-associated protein N",
  "term_id": "GO:0005737"
}